{
  "gene": "UniProtKB:O75628",
  "term_label": "GTP binding",
  "gene_name": "GTP-binding protein REM 1",
  "term_id": "GO:0005525",
  "gene_symbol": "REM1"
}